{
  "term_id": "GO:0043812",
  "gene_symbol": "SACM1L",
  "gene": "UniProtKB:Q9NTJ5",
  "term_label": "phosphatidylinositol-4-phosphate phosphatase activity",
  "gene_name": "Phosphatidylinositol-3-phosphatase SAC1"
}